glomerular mesangial cell differentiation [GO:0072008] (biological process) Relationships: is a type of GO:0035850; is_a mesangial cell differentiation [GO:0072007]; is part of glomerular mesangium development [GO:0072109] Subtypes: mesonephric glomerular mesangial cell differentiation [GO:0061259], metanephric glomerular mesangial cell differentiation [GO:0072254] Definition: The process in which relatively unspecialized cells acquire specialized structural and/or functional features that characterize the glomerular mesangial cells of the kidney as it progresses from its formation to the mature state. Sources: GOC:mtg_kidney_jan10